{
  "gene_symbol": "KDM2B",
  "gene": "UniProtKB:Q8NHM5",
  "term_label": "Unknown cellular component",
  "gene_name": "Lysine-specific demethylase 2B",
  "term_id": "UNKNOWN:0003"
}